flavonoid metabolic process [GO:0009812] (BP) Subtypes: flavonoid biosynthetic process [GO:0009813], GO:0046275, anthocyanin-containing compound metabolic process [GO:0046283], flavone metabolic process [GO:0051552], cyanidin 3-O-glucoside metabolic process [GO:1901038] Also known as: flavonoid metabolism Sources: GOC:tair_curators, ISBN:0198547684 Relationships: is a type of metabolic process [GO:0008152] Definition: The chemical reactions and pathways involving flavonoids, a group of water-soluble phenolic derivatives containing a flavan skeleton including flavones, flavonols and flavanoids, and anthocyanins.